{
  "term_label": "positive regulation of sodium ion export across plasma membrane",
  "gene_name": "FXYD domain-containing ion transport regulator 7",
  "term_id": "GO:1903278",
  "gene": "UniProtKB:P58549",
  "gene_symbol": "FXYD7"
}